mesonephric mesangial cell differentiation [GO:0061260] (biological process) Relationships: is a type of cell differentiation involved in mesonephros development [GO:0061208]; is a type of GO:0072007 Subtypes: mesonephric glomerular mesangial cell differentiation [GO:0061259] Definition: The process in which relatively unspecialized cells acquire specialized structural and/or functional features that characterize the mesangial cells of the mesonephros as it progresses from its formation to the mature state. Sources: GOC:mtg_kidney_jan10